{
  "gene": "UniProtKB:P32239",
  "term_id": "GO:0008188",
  "gene_symbol": "CCKBR",
  "term_label": "neuropeptide receptor activity",
  "gene_name": "Gastrin_cholecystokinin type B receptor"
}